{
  "gene": "UniProtKB:Q86WV6",
  "term_id": "GO:0016239",
  "term_label": "positive regulation of macroautophagy",
  "gene_name": "Stimulator of interferon genes protein",
  "gene_symbol": "STING1"
}